{
  "term_label": "external side of plasma membrane",
  "gene_name": "C-C chemokine receptor type 3",
  "gene_symbol": "CCR3",
  "term_id": "GO:0009897",
  "gene": "UniProtKB:P51677"
}